{
  "gene_symbol": "PXK",
  "term_id": "GO:0050804",
  "term_label": "modulation of chemical synaptic transmission",
  "gene_name": "PX domain-containing protein kinase-like protein",
  "gene": "UniProtKB:Q7Z7A4"
}